{
  "gene": "UniProtKB:A1L4H1",
  "term_id": "GO:0031012",
  "gene_symbol": "SSC5D",
  "gene_name": "Soluble scavenger receptor cysteine-rich domain-containing protein SSC5D",
  "term_label": "extracellular matrix"
}